modulation by host of RNA binding by virus [GO:1990968] (BP) Definition: A process in which a host organism modulates the frequency, rate or extent of a viral gene product binding to RNA. Also known as: modulation by host of viral protein:RNA interaction References: PMID:25116364 Sources: GOC:PARL, GOC:bf Relationships: is a type of modulation by host of viral molecular function [GO:0044868] Note: Note that the bound RNA may originate from the virus or another organism, including the host.